UTP catabolic process [GO:0046052] (biological process) Sources: GOC:go_curators Definition: The chemical reactions and pathways resulting in the breakdown of UTP, uridine (5'-)triphosphate. Relationships: is a type of pyrimidine ribonucleoside triphosphate catabolic process [GO:0009210]; is a type of pyrimidine ribonucleotide catabolic process [GO:0009222]; is a type of UTP metabolic process [GO:0046051] Also known as: UTP breakdown, UTP catabolism, UTP degradation, UTP hydrolysis